{
  "gene_symbol": "ALG14",
  "term_label": "Unknown molecular function",
  "term_id": "UNKNOWN:0001",
  "gene_name": "UDP-N-acetylglucosamine transferase subunit ALG14 homolog",
  "gene": "UniProtKB:Q96F25"
}